regulation of translational initiation by tRNA modification [GO:1990983] (biological process) Definition: A process in which translation initiation is regulated by post-translation modifications of a tRNA molecule. References: PMID:27745969 Also known as: tRNA demethylation Relationships: is a type of tRNA modification [GO:0006400]; is a type of regulation of translational initiation [GO:0006446]